{
  "gene_name": "Serine_threonine-protein kinase PDIK1L",
  "gene": "UniProtKB:Q8N165",
  "term_label": "negative regulation of G2/MI transition of meiotic cell cycle",
  "term_id": "GO:0110031",
  "gene_symbol": "PDIK1L"
}